{
  "term_label": "nerve growth factor receptor binding",
  "gene": "UniProtKB:P34130",
  "gene_symbol": "NTF4",
  "term_id": "GO:0005163",
  "gene_name": "Neurotrophin-4"
}